flower morphogenesis [GO:0048439] (BP) Sources: GOC:go_curators Definition: The process in which the anatomical structures of the flower are generated and organized. Relationships: is a type of developmental process involved in reproduction [GO:0003006]; is a type of shoot system morphogenesis [GO:0010016]; is a type of post-embryonic plant morphogenesis [GO:0090698]; is part of flower development [GO:0009908]